{
  "gene": "UniProtKB:Q92828",
  "term_id": "GO:0005884",
  "term_label": "actin filament",
  "gene_name": "Coronin-2A",
  "gene_symbol": "CORO2A"
}